G protein-coupled receptor heterodimeric complex [GO:0038039] (cellular component) References: PMID:16109836, PMID:20150590 Sources: GOC:al, GOC:bf Also known as: G-protein coupled receptor heterodimer, G-protein coupled receptor heterodimeric complex, GPCR heterodimer Definition: A protein complex that contains two G protein-coupled receptors (GPCRs) of different subtypes. Formation of a GPCR heterodimer may alter the functional property of the GPCR. Relationships: is a type of GO:0038037